{
  "gene_symbol": "NFE2L1",
  "gene": "UniProtKB:Q14494",
  "gene_name": "Endoplasmic reticulum membrane sensor NFE2L1",
  "term_id": "GO:0000981",
  "term_label": "DNA-binding transcription factor activity, RNA polymerase II-specific"
}